{
  "gene_symbol": "CA12",
  "term_label": "plasma membrane",
  "gene_name": "Carbonic anhydrase 12",
  "gene": "UniProtKB:O43570",
  "term_id": "GO:0005886"
}